{
  "gene": "UniProtKB:P08648",
  "gene_symbol": "ITGA5",
  "term_label": "integrin-mediated signaling pathway",
  "gene_name": "Integrin alpha-5",
  "term_id": "GO:0007229"
}